{
  "term_label": "Unknown cellular component",
  "gene_symbol": "FAM215A",
  "term_id": "UNKNOWN:0003",
  "gene_name": "Uncharacterized protein FAM215A",
  "gene": "UniProtKB:Q9Y5M1"
}